{
  "term_id": "GO:0070914",
  "gene_symbol": "ERCC1",
  "term_label": "UV-damage excision repair",
  "gene_name": "DNA excision repair protein ERCC-1",
  "gene": "UniProtKB:P07992"
}